{
  "term_label": "negative regulation of canonical Wnt signaling pathway",
  "gene": "UniProtKB:P49841",
  "gene_symbol": "GSK3B",
  "gene_name": "Glycogen synthase kinase-3 beta",
  "term_id": "GO:0090090"
}